{
  "gene": "UniProtKB:Q8NHY2",
  "term_id": "GO:0061630",
  "gene_symbol": "COP1",
  "gene_name": "E3 ubiquitin-protein ligase COP1",
  "term_label": "ubiquitin protein ligase activity"
}